{
  "term_id": "UNKNOWN:0002",
  "gene_symbol": "SH2D3C",
  "gene_name": "SH2 domain-containing protein 3C",
  "term_label": "Unknown biological process",
  "gene": "UniProtKB:Q8N5H7"
}